{
  "term_label": "positive regulation of cell migration",
  "gene_symbol": "CCL4L1",
  "gene_name": "C-C motif chemokine 4-like",
  "term_id": "GO:0030335",
  "gene": "UniProtKB:Q8NHW4"
}